{
  "term_id": "UNKNOWN:0001",
  "gene_name": "14-3-3 protein zeta_delta",
  "gene_symbol": "YWHAZ",
  "gene": "UniProtKB:P63104",
  "term_label": "Unknown molecular function"
}